floral whorl development [GO:0048438] (biological process) Sources: GOC:PO_curators, GOC:dph, GOC:go_curators, GOC:tb, PO:0025023 Also known as: collective phyllome structure development Subtypes: flower calyx development [GO:0048464], corolla development [GO:0048465], GO:0048466, GO:0048467, perianth development [GO:0090428] Relationships: is a type of developmental process involved in reproduction [GO:0003006]; is a type of GO:0048856; is part of flower development [GO:0009908] Definition: The process whose specific outcome is the progression of a floral whorl over time, from its formation to the mature structure. A floral whorl is a circular arrangement of parts of a flower arising from a stem of a plant. Note: Consider instead annotating to one of the more specific child terms, or to 'floral organ development ; GO:0048438' or one of its child terms.